nicotinate nucleotide biosynthetic process from tryptophan [GO:0019356] (biological process) Sources: GOC:go_curators Also known as: nicotinate nucleotide anabolism from tryptophan, nicotinate nucleotide formation from tryptophan, nicotinate nucleotide synthesis from tryptophan Definition: The chemical reactions and pathways resulting in the formation of nicotinate nucleotide from other compounds, including tryptophan. Relationships: is a type of aromatic amino acid metabolic process [GO:0009072]; is a type of GO:0019357; is a type of indole-containing compound metabolic process [GO:0042430]; is a type of alpha-amino acid metabolic process [GO:1901605]